diazepam binding [GO:0050809] (molecular function) Also known as: Valium binding, diazepam binding inhibitor activity Definition: Binding to diazepam, one of the most widely used benzodiazepine drugs. It is used as an anti-anxiety-hypnotic agent and has the proprietary name Valium. Sources: ISBN:0198506732 Relationships: is a type of binding [GO:0005488]